{
  "term_id": "GO:0051453",
  "gene": "UniProtKB:Q5TAH2",
  "gene_symbol": "SLC9C2",
  "term_label": "regulation of intracellular pH",
  "gene_name": "Sodium_hydrogen exchanger 11"
}